{
  "gene": "UniProtKB:P21709",
  "term_label": "receptor complex",
  "term_id": "GO:0043235",
  "gene_name": "Ephrin type-A receptor 1",
  "gene_symbol": "EPHA1"
}